D-glucose transmembrane transport [GO:1904659] (biological process) References: PMID:9090050 Sources: GOC:TermGenie, GO_REF:0000069 Also known as: glucose transmembrane transport, glucose transport Definition: The process in which D-glucose is transported across a membrane. Relationships: is a type of hexose transmembrane transport [GO:0008645] Subtypes: GO:0035623, GO:0046323, D-glucose import across plasma membrane [GO:0098708] Regulation: regulated by regulation of D-glucose transmembrane transport [GO:0010827]; positively regulated by positive regulation of D-glucose transmembrane transport [GO:0010828]; negatively regulated by negative regulation of D-glucose transmembrane transport [GO:0010829]